{
  "gene": "UniProtKB:Q0VAA5",
  "gene_symbol": "PLCXD2",
  "gene_name": "PI-PLC X domain-containing protein 2",
  "term_id": "UNKNOWN:0003",
  "term_label": "Unknown cellular component"
}